{
  "term_label": "autophagosome membrane",
  "term_id": "GO:0000421",
  "gene_name": "Tectonin beta-propeller repeat-containing protein 1",
  "gene": "UniProtKB:Q7Z6L1",
  "gene_symbol": "TECPR1"
}